{
  "gene_symbol": "FBXO6",
  "term_label": "ubiquitin protein ligase activity",
  "gene_name": "F-box only protein 6",
  "gene": "UniProtKB:Q9NRD1",
  "term_id": "GO:0061630"
}